{
  "gene_symbol": "GAL3ST2",
  "term_label": "galactose 3-O-sulfotransferase activity",
  "gene": "UniProtKB:Q9H3Q3",
  "term_id": "GO:0050694",
  "gene_name": "Galactose-3-O-sulfotransferase 2"
}